{
  "term_label": "mRNA binding",
  "gene_name": "RNA-binding protein 47",
  "gene_symbol": "RBM47",
  "term_id": "GO:0003729",
  "gene": "UniProtKB:A0AV96"
}